{
  "gene_symbol": "FSD1L",
  "gene": "UniProtKB:Q9BXM9",
  "term_id": "UNKNOWN:0003",
  "gene_name": "FSD1-like protein",
  "term_label": "Unknown cellular component"
}